orthokinesis [GO:0042467] (biological process) Definition: The movement of a cell or organism in response to a stimulus in which the speed or frequency of movement is increased or decreased. References: PMID:8207088 Sources: GOC:jl Relationships: is a type of kinesis [GO:0042465]